{
  "gene_symbol": "STIMATE",
  "term_label": "cortical endoplasmic reticulum",
  "gene_name": "Store-operated calcium entry regulator STIMATE",
  "term_id": "GO:0032541",
  "gene": "UniProtKB:Q86TL2"
}